peptidyl-proline hydroxylation [GO:0019511] (biological process) Definition: The hydroxylation of peptidyl-proline to form peptidyl-hydroxyproline. Sources: GOC:mah Relationships: is a type of protein hydroxylation [GO:0018126]; is a type of peptidyl-proline modification [GO:0018208] Subtypes: peptidyl-proline di-hydroxylation [GO:0018188], peptidyl-proline hydroxylation to 3-hydroxy-L-proline [GO:0018400], peptidyl-proline hydroxylation to 4-hydroxy-L-proline [GO:0018401]